{
  "term_label": "cell surface",
  "gene_symbol": "ITGAD",
  "gene": "UniProtKB:Q13349",
  "gene_name": "Integrin alpha-D",
  "term_id": "GO:0009986"
}